{
  "term_label": "regulation of transcription by RNA polymerase II",
  "gene_name": "Max dimerization protein 1",
  "term_id": "GO:0006357",
  "gene": "UniProtKB:Q05195",
  "gene_symbol": "MXD1"
}